GTP biosynthetic process [GO:0006183] (biological process) Definition: The chemical reactions and pathways resulting in the formation of GTP, guanosine triphosphate. Relationships: is a type of GO:0009152; is_a purine ribonucleoside triphosphate biosynthetic process [GO:0009206]; is a type of GTP metabolic process [GO:0046039] Also known as: GTP anabolism, GTP biosynthesis, GTP formation, GTP synthesis Sources: ISBN:0198506732